{
  "term_label": "intra-Golgi vesicle-mediated transport",
  "gene": "UniProtKB:P48553",
  "term_id": "GO:0006891",
  "gene_name": "Trafficking protein particle complex subunit 10",
  "gene_symbol": "TRAPPC10"
}